{
  "gene_symbol": "ZNF433",
  "gene_name": "Zinc finger protein 433",
  "term_id": "GO:0005634",
  "gene": "UniProtKB:Q8N7K0",
  "term_label": "nucleus"
}